epithelial-mesenchymal cell signaling involved in lung development [GO:0061111] (biological process) Sources: GOC:dph Definition: Any process that results in the transfer of information from an epithelial cell to a mesenchymal cell and contributes to the progression of the lung over time from its initial formation to the mature organ. Also known as: epithelial-mesenchymal cell signalling involved in lung development Relationships: is_a cell-cell signaling involved in lung development [GO:0060495]; is a type of epithelial-mesenchymal cell signaling [GO:0060684]